positive regulation of large conductance calcium-activated potassium channel activity [GO:1902608] (BP) Definition: Any process that activates or increases the frequency, rate or extent of large conductance calcium-activated potassium channel activity. Relationships: is a type of positive regulation of cation channel activity [GO:2001259]; positively regulates large conductance calcium-activated potassium channel activity [GO:0060072] References: PMID:23407708 Sources: GOC:TermGenie, GO_REF:0000059 Also known as: positive regulation of BK KCa channels, positive regulation of BK calcium-activated potassium channel activity, positive regulation of large conductance KCa channels, up regulation of BK KCa channels, up regulation of BK calcium-activated potassium channel activity, up regulation of large conductance KCa channels, up regulation of large conductance calcium-activated potassium channel activity, up-regulation of BK KCa channels, up-regulation of BK calcium-activated potassium channel activity, up-regulation of large conductance KCa channels, up-regulation of large conductance calcium-activated potassium channel activity, upregulation of BK KCa channels, upregulation of BK calcium-activated potassium channel activity, upregulation of large conductance KCa channels, upregulation of large conductance calcium-activated potassium channel activity, activation of BK KCa channels, activation of BK calcium-activated potassium channel activity, activation of large conductance KCa channels, activation of large conductance calcium-activated potassium channel activity, activation of BK channel activity, positive regulation of BK channel activity, up regulation of BK channel activity, up-regulation of BK channel activity, upregulation of BK channel activity